{
  "term_label": "DNA-binding transcription factor activity, RNA polymerase II-specific",
  "term_id": "GO:0000981",
  "gene_symbol": "ZNF81",
  "gene": "UniProtKB:P51508",
  "gene_name": "Zinc finger protein 81"
}